{
  "gene_symbol": "PPP1R13L",
  "gene": "UniProtKB:Q8WUF5",
  "term_id": "GO:0006357",
  "term_label": "regulation of transcription by RNA polymerase II",
  "gene_name": "RelA-associated inhibitor"
}